{
  "gene_name": "Dolichyl-phosphate beta-glucosyltransferase",
  "term_label": "dolichol-linked oligosaccharide biosynthetic process",
  "gene_symbol": "ALG5",
  "term_id": "GO:0006488",
  "gene": "UniProtKB:Q9Y673"
}